{
  "gene_symbol": "MRPL36",
  "gene_name": "Large ribosomal subunit protein bL36m",
  "gene": "UniProtKB:Q9P0J6",
  "term_label": "Unknown biological process",
  "term_id": "UNKNOWN:0002"
}